{
  "term_id": "GO:0007030",
  "term_label": "Golgi organization",
  "gene_name": "Golgin subfamily A member 8M",
  "gene": "UniProtKB:H3BSY2",
  "gene_symbol": "GOLGA8M"
}